response to azide [GO:0097184] (biological process) Relationships: is a type of response to nitrogen compound [GO:1901698] Subtypes: cellular response to azide [GO:0097185] References: PMID:16846222 Sources: GOC:yaf Definition: Any process that results in a change in state or activity of a cell or an organism (in terms of movement, secretion, enzyme production, gene expression, etc.) as a result of an azide stimulus.